visual learning [GO:0008542] (biological process) Relationships: is a type of visual behavior [GO:0007632]; is a type of GO:0008306 Sources: GOC:jid, ISBN:0582227089 Definition: Any process in an organism in which a change in behavior of an individual occurs in response to repeated exposure to a visual cue. Also known as: spatial learning